{
  "gene_symbol": "CD1D",
  "gene_name": "Antigen-presenting glycoprotein CD1d",
  "gene": "UniProtKB:P15813",
  "term_id": "GO:0048007",
  "term_label": "antigen processing and presentation, exogenous lipid antigen via MHC class Ib"
}